{
  "gene": "UniProtKB:Q16204",
  "gene_symbol": "CCDC6",
  "term_label": "Unknown molecular function",
  "term_id": "UNKNOWN:0001",
  "gene_name": "Coiled-coil domain-containing protein 6"
}